{
  "term_label": "cytoplasm",
  "gene": "UniProtKB:Q96NL8",
  "gene_symbol": "CFAP418",
  "term_id": "GO:0005737",
  "gene_name": "Cilia- and flagella-associated protein 418"
}